{
  "gene_name": "Protein LTV1 homolog",
  "gene": "UniProtKB:Q96GA3",
  "term_id": "GO:0005829",
  "term_label": "cytosol",
  "gene_symbol": "LTV1"
}